alphaIIb-beta3 integrin-CD9 complex [GO:0071085] (cellular component) References: PMID:10429193 Definition: A protein complex that consists of an alphaIIb-beta3 integrin complex bound to the cell surface protein CD9. Also known as: ITGA2b-ITGB3-CD9 complex Relationships: is a type of GO:0098797